{
  "gene_symbol": "METTL18",
  "term_label": "protein-L-histidine N-tele-methyltransferase activity",
  "gene": "UniProtKB:O95568",
  "term_id": "GO:0018064",
  "gene_name": "Histidine protein methyltransferase 1 homolog"
}